RNA polymerase II CTD heptapeptide repeat Y1 phosphatase activity [GO:0180004] (molecular function) Also known as: RNA polymerase II C-terminal domain Y1 phosphatase activity Definition: Catalysis of the reaction: RNA polymerase II large subunit CTD heptapeptide repeat--phospho-L-tyrosine (consensus YSPTSPS)(position 1) + H2O = RNA polymerase II large subunit + phosphate. Relationships: is a type of GO:0008420 References: PMID:22622228